{
  "gene_symbol": "FANCB",
  "gene": "UniProtKB:Q8NB91",
  "term_label": "Unknown molecular function",
  "term_id": "UNKNOWN:0001",
  "gene_name": "Fanconi anemia group B protein"
}